{
  "term_label": "monoatomic ion homeostasis",
  "gene_name": "Solute carrier family 4 member 11",
  "gene": "UniProtKB:Q8NBS3",
  "term_id": "GO:0050801",
  "gene_symbol": "SLC4A11"
}